{
  "gene_name": "Bargin",
  "term_id": "GO:0051058",
  "term_label": "negative regulation of small GTPase mediated signal transduction",
  "gene_symbol": "BARGIN",
  "gene": "UniProtKB:Q6ZT62"
}